epicardium-derived cardiac vascular smooth muscle cell development [GO:0060984] (biological process) Relationships: is a type of cardiac vascular smooth muscle cell development [GO:0060948]; is part of epicardium-derived cardiac vascular smooth muscle cell differentiation [GO:0060983] Definition: The process whose specific outcome is the progression of a cardiac vascular smooth muscle cell that was derived from the epicardium over time, from its formation to the mature state. Sources: GOC:mtg_heart